{
  "term_label": "tRNA-splicing ligase complex",
  "gene_name": "RNA-splicing ligase RtcB homolog",
  "gene_symbol": "RTCB",
  "gene": "UniProtKB:Q9Y3I0",
  "term_id": "GO:0072669"
}